anterograde dendritic transport of neurotransmitter receptor complex [GO:0098971] (biological process) Sources: GOC:dos Relationships: is a type of receptor localization to synapse [GO:0097120]; is a type of anterograde dendritic transport [GO:0098937] Definition: The directed movement of a neurotransmitter receptor complex along microtubules in nerve cell dendrites towards the postsynapse.